{
  "gene": "UniProtKB:O14613",
  "term_label": "plasma membrane",
  "gene_name": "Cdc42 effector protein 2",
  "gene_symbol": "CDC42EP2",
  "term_id": "GO:0005886"
}